{
  "gene_name": "Endothelial cell-specific molecule 1",
  "gene": "UniProtKB:Q9NQ30",
  "gene_symbol": "ESM1",
  "term_label": "Unknown cellular component",
  "term_id": "UNKNOWN:0003"
}